cytochrome b6f complex assembly [GO:0010190] (biological process) Definition: Formation of cytochrome b6f complex, a complex that transfers electrons from reduced plastoquinone to oxidized plastocyanin and translocates protons from the stroma to the lumen, by the aggregation, arrangement and bonding together of its constituents. Relationships: is a type of cytochrome complex assembly [GO:0017004] Sources: GOC:tb Also known as: cytochrome b6f complex biogenesis